{
  "term_id": "GO:0000455",
  "gene_symbol": "RPUSD3",
  "gene": "UniProtKB:Q6P087",
  "term_label": "enzyme-directed rRNA pseudouridine synthesis",
  "gene_name": "Mitochondrial mRNA pseudouridine synthase RPUSD3"
}